CUE1-UBC7 ubiquitin-conjugating enzyme complex [GO:1990389] (cellular component) Relationships: is a type of GO:0000835; is a type of ubiquitin conjugating enzyme complex [GO:0031371] Definition: A protein complex capable of ubiquitin-conjugating enzyme activity during ER-associated protein degradation (ERAD). In S. cerevisiae, UBC7 is the ubiquitin-conjugating enzyme (E2) and requires binding to the ER surface by CUE1. Note: An example of this is UBC7 in Saccharomyces cerevisiae (Q02159) in PMID:16179953 (inferred from direct assay). References: PMID:23028185 Sources: GOC:bhm Also known as: CUE1-UBC7 ubiquitin-conjugating enzyme (E2)